phosphatidylcholine biosynthesis from phosphoryl-ethanolamine via CDP-N-methylethanolamine [GO:0070833] (biological process) Definition: The phosphatidylcholine biosynthetic process that begins with an initial N-methylation with phospho-base phosphoethanolamine, followed by two downstream N-methylations on phosphatidyl-bases, phosphatidyl-N-methylethanolamine and phosphatidyl-N-dimethylethanolamine. The process ends with the conversion of a phosphatidyl-N-dimethylethanolamine to a phosphatidylcholine. Relationships: is a type of phosphatidylcholine biosynthetic process [GO:0006656] Sources: MetaCyc:PWY4FS-3